{
  "term_label": "heme binding",
  "gene": "UniProtKB:P51589",
  "term_id": "GO:0020037",
  "gene_name": "Cytochrome P450 2J2",
  "gene_symbol": "CYP2J2"
}